tube closure [GO:0060606] (biological process) Definition: Creation of the central hole of a tube in an anatomical structure by sealing the edges of an epithelial fold. Relationships: is a type of tube formation [GO:0035148] Sources: GOC:dph Subtypes: neural tube closure [GO:0001843], closure of embryonic heart tube [GO:0003153], GO:0060879, anterior neural tube closure [GO:0061713]